phospholipid efflux [GO:0033700] (biological process) Regulation: regulated by GO:1902994; RO_0002213 by GO:1902995; RO_0002212 by negative regulation of phospholipid efflux [GO:1902999] Definition: The directed movement of a phospholipid out of a cell or organelle. Also known as: phospholipid export Relationships: is a type of phospholipid transport [GO:0015914] Sources: GOC:mah